{
  "gene_symbol": "BIN1",
  "term_label": "phospholipid binding",
  "gene": "UniProtKB:O00499",
  "term_id": "GO:0005543",
  "gene_name": "Myc box-dependent-interacting protein 1"
}